{
  "term_id": "GO:0032154",
  "gene_symbol": "RAB11FIP4",
  "gene_name": "Rab11 family-interacting protein 4",
  "term_label": "cleavage furrow",
  "gene": "UniProtKB:Q86YS3"
}